{
  "gene_symbol": "ZBTB2",
  "gene_name": "Zinc finger and BTB domain-containing protein 2",
  "term_id": "GO:0001227",
  "term_label": "DNA-binding transcription repressor activity, RNA polymerase II-specific",
  "gene": "UniProtKB:Q8N680"
}